regulation of cell growth by extracellular stimulus [GO:0001560] (biological process) Definition: Any process in which external signals modulate the frequency, rate or extent of cell growth, the irreversible increase in size of a cell over time. Sources: GOC:dph Also known as: interpretation of external signals that regulate cell growth, regulation of cell growth by detection of exogenous stimulus, regulation of cell growth by sensing of exogenous stimulus, regulation of growth by exogenous signal, regulation of growth by exogenous stimuli, regulation of growth by exogenous stimulus, regulation of growth by external signal, regulation of growth by external stimuli, regulation of growth by external stimulus Relationships: is a type of regulation of cell growth [GO:0001558]; is part of cellular response to stimulus [GO:0051716]